{
  "gene_symbol": "FAAH",
  "gene": "UniProtKB:O00519",
  "term_label": "Unknown cellular component",
  "term_id": "UNKNOWN:0003",
  "gene_name": "Fatty-acid amide hydrolase 1"
}